interleukin-9-mediated signaling pathway [GO:0038113] (BP) Sources: GOC:nhn, GOC:signaling Also known as: IL-9-mediated signaling pathway, interleukin-9-mediated signalling pathway Definition: The series of molecular signals initiated by interleukin-9 binding to its receptor on the surface of a target cell, and ending with the regulation of a downstream cellular process, e.g. transcription. Relationships: is a type of cytokine-mediated signaling pathway [GO:0019221]; is part of cellular response to interleukin-9 [GO:0071355]